positive regulation of catecholamine uptake involved in synaptic transmission [GO:0051944] (biological process) Sources: GOC:ai, GOC:dph, GOC:tb Definition: Any process that activates, maintains or increases the frequency, rate or extent of the directed movement of catecholamine neurotransmitters into a neuron or glial cell. Subtypes: positive regulation of dopamine uptake involved in synaptic transmission [GO:0051586] Relationships: is a type of positive regulation of neurotransmitter uptake [GO:0051582]; is a type of regulation of catecholamine uptake involved in synaptic transmission [GO:0051940]; is_a positive regulation of amine transport [GO:0051954]; positively regulates catecholamine uptake involved in synaptic transmission [GO:0051934] Also known as: positive regulation of catecholamine uptake during transmission of nerve impulse, positive regulation of catecholamine neurotransmitter reuptake, positive regulation of catecholamine neurotransmitter uptake, up regulation of catecholamine uptake during transmission of nerve impulse, up-regulation of catecholamine uptake during transmission of nerve impulse, upregulation of catecholamine uptake during transmission of nerve impulse, activation of catecholamine uptake during transmission of nerve impulse, stimulation of catecholamine uptake during transmission of nerve impulse